heparosan-N-sulfate-glucuronate 5-epimerase activity [GO:0047464] (molecular function) Sources: EC:5.1.3.17, MetaCyc:5.1.3.17-RXN Relationships: is a type of GO:0016857 Definition: Catalysis of the reaction: (heparosan-N-sulfate)(n) = (heparan-N-sulfate)(n). Converts D-glucosyluronate residues to L-iduronate residues. Also known as: heparosan-N-sulphate-glucuronate 5-epimerase activity, C-5 uronosyl epimerase activity, D-glucuronyl C-5 epimerase activity, heparosan epimerase activity, heparosan-N-sulfate-D-glucuronosyl 5-epimerase activity, poly[(1,4)-beta-D-glucuronosyl-(1,4)-N-sulfo-alpha-D-glucosaminyl] glucurono-5-epimerase activity, polyglucuronate epimerase activity